{
  "term_label": "Unknown cellular component",
  "gene_name": "Uncharacterized protein C11orf16",
  "gene": "UniProtKB:Q9NQ32",
  "term_id": "UNKNOWN:0003",
  "gene_symbol": "C11orf16"
}